{
  "gene_symbol": "SUMF1",
  "gene_name": "Formylglycine-generating enzyme",
  "term_label": "Unknown biological process",
  "term_id": "UNKNOWN:0002",
  "gene": "UniProtKB:Q8NBK3"
}